host-mediated suppression of viral genome replication [GO:0044828] (biological process) Definition: A process in which a host organism interferes with, inhibits or disrupts viral genome replication. Sources: GOC:jl Also known as: negative regulation by host of viral genome replication Relationships: is a type of GO:0044788; negatively regulates viral genome replication [GO:0019079]